{
  "term_id": "UNKNOWN:0001",
  "term_label": "Unknown molecular function",
  "gene_symbol": "Q6ZUT4",
  "gene_name": "Putative uncharacterized protein FLJ43343",
  "gene": "UniProtKB:Q6ZUT4"
}